diphosphoinositol pentakisphosphate kinase activity [GO:0000829] (molecular function) References: PMID:16429326 Sources: GOC:elh Definition: Catalysis of the reaction: ATP + diphospho-1D-myo-inositol-pentakisphosphate = ADP + bis(diphospho)-1D-myo-inositol-tetrakisphosphate. The isomeric configurations of the diphospho-1D-myo-inositol-pentakisphosphate (PP-IP5) and bis(diphospho)-1D-myo-inositol-tetrakisphosphate (bis-PP-IP4) are unknown. Subtypes: 5-diphosphoinositol pentakisphosphate 4-kinase activity [GO:0000833], 5-diphosphoinositol pentakisphosphate 6-kinase activity [GO:0000834], diphosphoinositol pentakisphosphate 5-kinase activity [GO:0033200], GO:0033857 Also known as: PP-IP5 kinase activity, inositol heptakisphosphate kinase activity Relationships: is a type of GO:0016776; is a type of inositol phosphate kinase activity [GO:0180030]